{
  "term_label": "ubiquitin-dependent protein catabolic process",
  "gene_symbol": "RLIM",
  "gene_name": "E3 ubiquitin-protein ligase RLIM",
  "gene": "UniProtKB:Q9NVW2",
  "term_id": "GO:0006511"
}